regulation of intralumenal vesicle formation [GO:1905365] (biological process) Subtypes: negative regulation of intralumenal vesicle formation [GO:1905366], positive regulation of intralumenal vesicle formation [GO:1905367] References: PMID:26911690 Sources: GOC:PARL, GOC:TermGenie, GOC:bc, GO_REF:0000058 Also known as: regulation of endosome membrane budding Relationships: is a type of regulation of endosome organization [GO:1904978]; regulates intralumenal vesicle formation [GO:0070676] Definition: Any process that modulates the frequency, rate or extent of intralumenal vesicle formation.